{
  "term_id": "GO:0071222",
  "gene_symbol": "CD80",
  "gene": "UniProtKB:P33681",
  "gene_name": "T-lymphocyte activation antigen CD80",
  "term_label": "cellular response to lipopolysaccharide"
}